{
  "gene": "UniProtKB:Q8N257",
  "gene_name": "Histone H2B type 3-B",
  "term_label": "antimicrobial humoral immune response mediated by antimicrobial peptide",
  "term_id": "GO:0061844",
  "gene_symbol": "H2BC26"
}